{
  "term_id": "GO:0004957",
  "gene": "UniProtKB:P35408",
  "gene_name": "Prostaglandin E2 receptor EP4 subtype",
  "term_label": "prostaglandin E receptor activity",
  "gene_symbol": "PTGER4"
}